regulation of emericellin biosynthetic process [GO:1900834] (BP) Sources: GOC:TermGenie, GOC:di Subtypes: negative regulation of emericellin biosynthetic process [GO:1900835], positive regulation of emericellin biosynthetic process [GO:1900836] Relationships: is a type of regulation of xanthone-containing compound biosynthetic process [GO:1900183]; is a type of GO:1900376; regulates emericellin biosynthetic process [GO:1900766] Definition: Any process that modulates the frequency, rate or extent of emericellin biosynthetic process. Also known as: regulation of emericellin anabolism, regulation of emericellin biosynthesis, regulation of emericellin formation, regulation of emericellin synthesis, regulation of Variecoxanthone B anabolism, regulation of Variecoxanthone B biosynthesis, regulation of Variecoxanthone B biosynthetic process, regulation of Variecoxanthone B formation, regulation of Variecoxanthone B synthesis